{
  "gene_symbol": "UBE2G1",
  "term_id": "GO:0043161",
  "gene": "UniProtKB:P62253",
  "gene_name": "Ubiquitin-conjugating enzyme E2 G1",
  "term_label": "proteasome-mediated ubiquitin-dependent protein catabolic process"
}